{
  "term_label": "telomere maintenance",
  "gene_name": "Bifunctional 3'-5' exonuclease_ATP-dependent helicase WRN",
  "gene": "UniProtKB:Q14191",
  "gene_symbol": "WRN",
  "term_id": "GO:0000723"
}